{
  "term_label": "tumor necrosis factor receptor binding",
  "gene": "UniProtKB:Q13077",
  "gene_symbol": "TRAF1",
  "term_id": "GO:0005164",
  "gene_name": "TNF receptor-associated factor 1"
}